{
  "gene_name": "Proteasome subunit beta type-7",
  "gene": "UniProtKB:Q99436",
  "gene_symbol": "PSMB7",
  "term_id": "GO:0005829",
  "term_label": "cytosol"
}